{
  "gene_name": "Tetratricopeptide repeat protein 39B",
  "term_id": "GO:0010874",
  "gene_symbol": "TTC39B",
  "gene": "UniProtKB:Q5VTQ0",
  "term_label": "regulation of cholesterol efflux"
}